alpha-cuprenene synthase activity [GO:0102885] (molecular function) Sources: EC:4.2.3.95, GOC:pz Definition: Catalysis of the reaction: 2-trans,6-trans-farnesyl diphosphate = (-)-alpha-cuprenene + diphosphoric acid. Relationships: is a type of GO:0016838